positive regulation of glucocorticoid catabolic process [GO:0031951] (biological process) Definition: Any process that activates or increases the frequency, rate or extent of the chemical reactions and pathways resulting in the breakdown of glucocorticoids. Relationships: is a type of regulation of glucocorticoid catabolic process [GO:0031949]; is a type of positive regulation of steroid metabolic process [GO:0045940]; is a type of positive regulation of lipid catabolic process [GO:0050996]; positively regulates glucocorticoid catabolic process [GO:0006713] Sources: GOC:mah Also known as: up regulation of glucocorticoid catabolic process, up-regulation of glucocorticoid catabolic process, upregulation of glucocorticoid catabolic process, activation of glucocorticoid catabolic process, stimulation of glucocorticoid catabolic process